{
  "gene_symbol": "CLPB",
  "term_label": "cellular response to heat",
  "term_id": "GO:0034605",
  "gene_name": "Mitochondrial disaggregase",
  "gene": "UniProtKB:Q9H078"
}